{
  "term_label": "positive regulation of long-term neuronal synaptic plasticity",
  "gene_symbol": "FXR1",
  "gene": "UniProtKB:P51114",
  "gene_name": "RNA-binding protein FXR1",
  "term_id": "GO:0048170"
}